PeBoW complex [GO:0070545] (cellular component) Definition: A protein complex that is involved in coordinating ribosome biogenesis with cell cycle progression. In human, it is composed of Pes1, Bop1, and WDR12; in Saccharomyces the proteins are known as Nop7p, Erb1 and Ytm1 respectively. Relationships: is a type of nuclear protein-containing complex [GO:0140513]; BFO_0000050 nucleolus [GO:0005730]; is part of 90S preribosome [GO:0030686] References: PMID:16043514, PMID:17353269 Sources: GOC:ab, GOC:mah